{
  "term_id": "GO:0043066",
  "term_label": "negative regulation of apoptotic process",
  "gene_symbol": "DSTYK",
  "gene_name": "Dual serine_threonine and tyrosine protein kinase",
  "gene": "UniProtKB:Q6XUX3"
}